larval development [GO:0002164] (BP) Subtypes: amphibian larval development [GO:0002117], nematode larval development [GO:0002119], instar larval development [GO:0002168] Definition: The process whose specific outcome is the progression of the larva over time, from its formation to the mature structure. The larva is the early, immature form of an that at birth or hatching is fundamentally unlike its parent and must metamorphose before assuming the adult characters. Sources: GOC:jid, ISBN:0877795088 Relationships: is a type of multicellular organism development [GO:0007275]; is a type of GO:0009791